positive regulation of nucleotide metabolic process [GO:0045981] (biological process) Relationships: is_a regulation of nucleotide metabolic process [GO:0006140]; is a type of positive regulation of phosphate metabolic process [GO:0045937]; is a type of GO:0062013; positively regulates GO:0009117 Subtypes: GO:0030810, positive regulation of nucleotide catabolic process [GO:0030813], positive regulation of purine nucleotide metabolic process [GO:1900544] Also known as: positive regulation of nucleotide metabolism, up regulation of nucleotide metabolic process, up-regulation of nucleotide metabolic process, upregulation of nucleotide metabolic process, activation of nucleotide metabolic process, stimulation of nucleotide metabolic process Definition: Any process that activates or increases the frequency, rate or extent of the chemical reactions and pathways involving nucleotides. Sources: GOC:go_curators